{
  "gene_name": "T cell receptor alpha variable 26-1",
  "gene": "UniProtKB:A0A087WT03",
  "term_id": "GO:0009617",
  "term_label": "response to bacterium",
  "gene_symbol": "TRAV26-1"
}